{
  "gene_name": "Hemoglobin subunit gamma-1",
  "gene": "UniProtKB:P69891",
  "term_label": "erythrocyte development",
  "gene_symbol": "HBG1",
  "term_id": "GO:0048821"
}